{
  "gene": "UniProtKB:P35346",
  "term_id": "GO:0004994",
  "term_label": "somatostatin receptor activity",
  "gene_name": "Somatostatin receptor type 5",
  "gene_symbol": "SSTR5"
}